plant-type vacuole [GO:0000325] (cellular component) Definition: A closed structure that is completely surrounded by a unit membrane, contains liquid, and retains the same shape regardless of cell cycle phase. An example of this structure is found in Arabidopsis thaliana. Also known as: vacuole, cell cycle-independent morphology Sources: GOC:mtg_sensu, ISBN:0815316208 Relationships: is a type of vacuole [GO:0005773] Subtypes: protein storage vacuole [GO:0000326], senescence-associated vacuole [GO:0010282], GO:0042807